{
  "gene_name": "Max dimerization protein 3",
  "gene": "UniProtKB:Q9BW11",
  "gene_symbol": "MXD3",
  "term_label": "DNA-binding transcription factor activity, RNA polymerase II-specific",
  "term_id": "GO:0000981"
}